{
  "gene": "UniProtKB:Q9GZR1",
  "gene_symbol": "SENP6",
  "gene_name": "Sentrin-specific protease 6",
  "term_id": "GO:0070139",
  "term_label": "SUMO-specific endopeptidase activity"
}